{
  "gene": "UniProtKB:Q9Y5Z0",
  "term_label": "amyloid-beta metabolic process",
  "gene_symbol": "BACE2",
  "term_id": "GO:0050435",
  "gene_name": "Beta-secretase 2"
}